{
  "gene_symbol": "LARS2",
  "term_label": "leucyl-tRNA aminoacylation",
  "gene_name": "Leucine--tRNA ligase, mitochondrial",
  "gene": "UniProtKB:Q15031",
  "term_id": "GO:0006429"
}